outer hair cell apoptotic process [GO:1905584] (biological process) Relationships: is a type of neuron apoptotic process [GO:0051402] Also known as: cochlear outer hair cell apoptotic process, cochlear outer hair cell apoptosis, outer hair cell apoptosis Definition: Any apoptotic process in an outer hair cell. Regulation: regulated by regulation of outer hair cell apoptotic process [GO:1905585]; RO_0002212 by negative regulation of outer hair cell apoptotic process [GO:1905586]; positively regulated by positive regulation of outer hair cell apoptotic process [GO:1905587] References: PMID:12062759, PMID:24472721 Sources: GOC:TermGenie, GO_REF:0000085